negative regulation of replicative senescence [GO:1904727] (biological process) References: PMID:23496142 Sources: GOC:BHF, GOC:BHF_miRNA, GOC:TermGenie, GOC:rph, GO_REF:0000058 Relationships: is a type of GO:0010948; is a type of regulation of replicative senescence [GO:1904726]; negatively regulates GO:0090399 Definition: Any process that stops, prevents or reduces the frequency, rate or extent of replicative senescence. Also known as: down regulation of replicative senescence, down-regulation of replicative senescence, downregulation of replicative senescence, inhibition of replicative senescence